type V protein secretion system complex [GO:0098046] (cellular component) Relationships: is a type of protein-containing complex [GO:0032991] Definition: A complex of proteins that permits the translocation of proteins across the outer membrane via a transmembrane pore, formed by a beta-barrel, into the extracellular milieu or directly into host cells; the secreted proteins contain all the information required for translocation of an effector molecule through the cell envelope. The type V secretion systems includes the autotransporters (type Va), the two-partner secretion system (type Vb) and the Oca family (type Vc). References: PMID:15119822, PMID:15590781 Sources: GOC:bf, GOC:bhm Note: Note that the type II protein secretion system complex does not include components of the Sec or Tat pathways. For components of these pathways, consider annotating to 'cell envelope Sec complex ; GO:0031522' or 'TAT protein translocation system complex ; GO:0033281'. Also known as: T5SS complex, autotransporter system complex